{
  "gene_symbol": "BTK",
  "gene": "UniProtKB:Q06187",
  "gene_name": "Tyrosine-protein kinase BTK",
  "term_label": "adaptive immune response",
  "term_id": "GO:0002250"
}